{
  "gene_symbol": "RRAS",
  "term_label": "Ras protein signal transduction",
  "gene_name": "Ras-related protein R-Ras",
  "gene": "UniProtKB:P10301",
  "term_id": "GO:0007265"
}